negative regulation of cell-substrate adhesion [GO:0010812] (biological process) Subtypes: GO:0001953, negative regulation of substrate adhesion-dependent cell spreading [GO:1900025], negative regulation of cell adhesion involved in single-species biofilm formation [GO:1900188], negative regulation of substrate-dependent cell migration, cell attachment to substrate [GO:1904236] Definition: Any process that decreases the frequency, rate or extent of cell-substrate adhesion. Cell-substrate adhesion is the attachment of a cell to the underlying substrate via adhesion molecules. Sources: GOC:dph, GOC:pf, GOC:tb Relationships: is a type of negative regulation of cell adhesion [GO:0007162]; is a type of regulation of cell-substrate adhesion [GO:0010810]; negatively regulates cell-substrate adhesion [GO:0031589]